{
  "gene_name": "BPI fold-containing family B member 1",
  "gene": "UniProtKB:Q8TDL5",
  "term_label": "Unknown molecular function",
  "term_id": "UNKNOWN:0001",
  "gene_symbol": "BPIFB1"
}